{
  "term_id": "GO:0005024",
  "term_label": "transforming growth factor beta receptor activity",
  "gene_name": "Transforming growth factor beta receptor type 3",
  "gene_symbol": "TGFBR3",
  "gene": "UniProtKB:Q03167"
}